{
  "term_label": "HIR complex",
  "gene_symbol": "HIRA",
  "gene_name": "Protein HIRA",
  "term_id": "GO:0000417",
  "gene": "UniProtKB:P54198"
}